{
  "term_id": "UNKNOWN:0001",
  "term_label": "Unknown molecular function",
  "gene": "UniProtKB:Q8IZ16",
  "gene_symbol": "SPACDR",
  "gene_name": "Sperm acrosome developmental regulator"
}